precorrin-6A reductase activity [GO:0016994] (molecular function) Sources: EC:1.3.1.54 Relationships: is a type of oxidoreductase activity, acting on the CH-CH group of donors, NAD or NADP as acceptor [GO:0016628] Definition: Catalysis of the reaction: precorrin-6B + NADP+ = precorrin-6A + NADPH + H+. Also known as: precorrin-6X reductase activity, precorrin-6B:NADP+ oxidoreductase activity, precorrin-6Y:NADP(+) oxidoreductase activity, precorrin-6Y:NADP+ oxidoreductase activity